{
  "gene": "UniProtKB:Q9Y450",
  "gene_symbol": "HBS1L",
  "term_id": "GO:0006412",
  "gene_name": "HBS1-like protein",
  "term_label": "translation"
}